{
  "term_label": "microtubule",
  "term_id": "GO:0005874",
  "gene": "UniProtKB:Q9Y496",
  "gene_symbol": "KIF3A",
  "gene_name": "Kinesin-like protein KIF3A"
}